regulation of natural killer cell proliferation [GO:0032817] (biological process) Relationships: is a type of regulation of natural killer cell activation [GO:0032814]; is a type of regulation of lymphocyte proliferation [GO:0050670]; regulates GO:0001787 Definition: Any process that modulates the frequency, rate or extent of natural killer cell proliferation. Sources: GOC:mah Also known as: regulation of NK cell proliferation Subtypes: negative regulation of natural killer cell proliferation [GO:0032818], positive regulation of natural killer cell proliferation [GO:0032819], regulation of natural killer cell proliferation involved in immune response [GO:0032820]